{
  "term_label": "negative regulation of DNA-templated transcription",
  "gene_symbol": "L3MBTL1",
  "gene": "UniProtKB:Q9Y468",
  "term_id": "GO:0045892",
  "gene_name": "Lethal(3)malignant brain tumor-like protein 1"
}